{
  "term_id": "GO:0030141",
  "gene_symbol": "KLK8",
  "gene_name": "Kallikrein-8",
  "term_label": "secretory granule",
  "gene": "UniProtKB:O60259"
}